{
  "term_label": "L-histidine transmembrane transporter activity",
  "gene": "UniProtKB:Q99624",
  "gene_symbol": "SLC38A3",
  "gene_name": "Sodium-coupled neutral amino acid transporter 3",
  "term_id": "GO:0005290"
}